{
  "term_label": "transcription cis-regulatory region binding",
  "gene": "UniProtKB:O15534",
  "term_id": "GO:0000976",
  "gene_symbol": "PER1",
  "gene_name": "Period circadian protein homolog 1"
}